regulation of extracellular exosome assembly [GO:1903551] (biological process) References: PMID:24105262 Sources: GOC:TermGenie, GO_REF:0000058 Subtypes: negative regulation of extracellular exosome assembly [GO:1903552], GO:1903553 Relationships: is a type of regulation of organelle assembly [GO:1902115]; RO_0002211 GO:0071971 Definition: Any process that modulates the frequency, rate or extent of extracellular vesicular exosome assembly. Also known as: regulation of extracellular vesicular exosome assembly